{
  "term_id": "GO:0060070",
  "term_label": "canonical Wnt signaling pathway",
  "gene_symbol": "BCL9",
  "gene": "UniProtKB:O00512",
  "gene_name": "B-cell CLL_lymphoma 9 protein"
}